{
  "gene_symbol": "TPRN",
  "gene": "UniProtKB:Q4KMQ1",
  "term_label": "Unknown molecular function",
  "gene_name": "Taperin",
  "term_id": "UNKNOWN:0001"
}